{
  "term_id": "GO:0051209",
  "term_label": "release of sequestered calcium ion into cytosol",
  "gene_symbol": "ITPR1",
  "gene": "UniProtKB:Q14643",
  "gene_name": "Inositol 1,4,5-trisphosphate receptor type 1"
}